{
  "gene_symbol": "PSMG2",
  "term_label": "proteasome assembly",
  "gene_name": "Proteasome assembly chaperone 2",
  "gene": "UniProtKB:Q969U7",
  "term_id": "GO:0043248"
}